cellular hypotonic response [GO:0071476] (biological process) Sources: GOC:mah Definition: Any process that results in a change in state or activity of a cell (in terms of movement, secretion, enzyme production, gene expression, etc.) as a result of detection of, or exposure to, a hypotonic environment, i.e. an environment with a lower concentration of solutes than the organism or cell. Subtypes: cellular hypotonic salinity response [GO:0071477] Relationships: is a type of hypotonic response [GO:0006971]; is a type of cellular response to osmotic stress [GO:0071470] Also known as: cellular hypo-osmotic response